neuropeptide binding [GO:0042923] (molecular function) Subtypes: GO:0042924 Definition: Interacting selectively and non-covalently and stoichiometrically with neuropeptides, peptides with direct synaptic effects (peptide neurotransmitters) or indirect modulatory effects on the nervous system (peptide neuromodulators). Relationships: is a type of peptide binding [GO:0042277] References: PMID:10414961, PMID:38337033